{
  "term_label": "plasma membrane",
  "gene_name": "Potassium channel subfamily K member 10",
  "gene": "UniProtKB:P57789",
  "term_id": "GO:0005886",
  "gene_symbol": "KCNK10"
}